geranylgeranyl diphosphate synthase activity [GO:0004311] (MF) Sources: RHEA:17653 Also known as: farnesyltranstransferase activity, geranylgeranyl pyrophosphate synthase activity, geranylgeranyl pyrophosphate synthetase activity, geranylgeranyl-PP synthetase activity, geranylgeranyl-diphosphate synthase activity, trans,trans-farnesyl-diphosphate:isopentenyl-diphosphate farnesyltranstransferase activity Relationships: is_a prenyl diphosphate synthase activity [GO:0120531] Note: The catalyzed reaction forms (free) geranylgeranyl diphosphate. There is no relationship between this activity and protein farnesyltransferase activity, GO:0004660, where the catalyzed reaction transfers a farnesyl group from farnesyl diphosphate to a target protein. Note that this term has a MetaCyc pathway reference as the pathway only has a single step. Definition: Catalysis of the reaction: (2E,6E)-farnesyl diphosphate + isopentenyl diphosphate = (2E,6E,10E)-geranylgeranyl diphosphate + diphosphate.